{
  "gene_symbol": "LZTFL1",
  "gene": "UniProtKB:Q9NQ48",
  "term_label": "negative regulation of protein localization to cilium",
  "term_id": "GO:1903565",
  "gene_name": "Leucine zipper transcription factor-like protein 1"
}